{
  "term_label": "nucleus",
  "gene_symbol": "EIF6",
  "term_id": "GO:0005634",
  "gene": "UniProtKB:P56537",
  "gene_name": "Eukaryotic translation initiation factor 6"
}